{
  "gene_symbol": "CYBB",
  "term_id": "GO:0005886",
  "term_label": "plasma membrane",
  "gene": "UniProtKB:P04839",
  "gene_name": "Cytochrome b-245 heavy chain"
}